{
  "gene_symbol": "SPIN4",
  "term_id": "GO:0005654",
  "term_label": "nucleoplasm",
  "gene_name": "Spindlin-4",
  "gene": "UniProtKB:Q56A73"
}